{
  "gene_symbol": "OR1L8",
  "gene_name": "Olfactory receptor 1L8",
  "term_label": "signal transduction",
  "term_id": "GO:0007165",
  "gene": "UniProtKB:Q8NGR8"
}